{
  "gene_symbol": "MTERF3",
  "gene_name": "Transcription termination factor 3, mitochondrial",
  "term_label": "Unknown molecular function",
  "term_id": "UNKNOWN:0001",
  "gene": "UniProtKB:Q96E29"
}